{
  "gene": "UniProtKB:Q9HD90",
  "term_label": "nucleus",
  "gene_symbol": "NEUROD4",
  "term_id": "GO:0005634",
  "gene_name": "Neurogenic differentiation factor 4"
}